kynurenate-7,8-dihydrodiol dehydrogenase activity [GO:0047114] (molecular function) Sources: EC:1.3.1.18, RHEA:22248 Also known as: 7,8-dihydro-7,8-dihydroxykynurenate dehydrogenase activity, 7,8-dihydro-7,8-dihydroxykynurenate:NAD+ oxidoreductase activity, 7,8-dihydroxykynurenic acid 7,8-diol dehydrogenase activity Definition: Catalysis of the reaction: 7,8-dihydro-7,8-dihydroxykynurenate + NAD+ = 7,8-dihydroxykynurenate + H+ + NADH. Relationships: is a type of oxidoreductase activity, acting on the CH-CH group of donors, NAD or NADP as acceptor [GO:0016628]